{
  "gene": "UniProtKB:Q6ICI0",
  "gene_name": "LHFPL tetraspan subfamily member 7 protein",
  "gene_symbol": "LHFPL7",
  "term_label": "Unknown biological process",
  "term_id": "UNKNOWN:0002"
}